{
  "term_label": "iron-sulfur cluster assembly",
  "gene": "UniProtKB:P38646",
  "term_id": "GO:0016226",
  "gene_name": "Stress-70 protein, mitochondrial",
  "gene_symbol": "HSPA9"
}